{
  "gene_name": "Muscarinic acetylcholine receptor M4",
  "term_id": "GO:0030425",
  "gene_symbol": "CHRM4",
  "term_label": "dendrite",
  "gene": "UniProtKB:P08173"
}